positive regulation of maintenance of bipolar cell polarity regulating cell shape [GO:0061361] (biological process) Definition: Any process that increases the frequency, rate or extent of maintenance of bipolar cell polarity regulating cell shape. Sources: GOC:dph Relationships: is a type of GO:2000115; is_a positive regulation of establishment or maintenance of bipolar cell polarity regulating cell shape [GO:2000247]; positively regulates GO:0061305